{
  "term_id": "GO:0000774",
  "gene_name": "BAG family molecular chaperone regulator 3",
  "gene": "UniProtKB:O95817",
  "gene_symbol": "BAG3",
  "term_label": "adenyl-nucleotide exchange factor activity"
}